{
  "term_id": "GO:0003677",
  "gene_symbol": "BCLAF1",
  "gene": "UniProtKB:Q9NYF8",
  "gene_name": "Bcl-2-associated transcription factor 1",
  "term_label": "DNA binding"
}